{
  "term_id": "GO:0005243",
  "term_label": "gap junction channel activity",
  "gene": "UniProtKB:Q969M2",
  "gene_symbol": "GJA10",
  "gene_name": "Gap junction alpha-10 protein"
}